{
  "gene_name": "Complement C1q tumor necrosis factor-related protein 2",
  "term_id": "UNKNOWN:0001",
  "term_label": "Unknown molecular function",
  "gene": "UniProtKB:Q9BXJ5",
  "gene_symbol": "C1QTNF2"
}